{
  "gene": "UniProtKB:P08686",
  "term_label": "steroid 21-monooxygenase activity",
  "gene_name": "Steroid 21-hydroxylase",
  "term_id": "GO:0004509",
  "gene_symbol": "CYP21A2"
}